{
  "term_label": "protein localization to plasma membrane",
  "gene_symbol": "FYB2",
  "term_id": "GO:0072659",
  "gene_name": "FYN-binding protein 2",
  "gene": "UniProtKB:Q5VWT5"
}